alphav-beta3 integrin-HMGB1 complex [GO:0035868] (cellular component) Relationships: is a type of plasma membrane protein complex [GO:0098797] Also known as: alphav-beta3 integrin-high mobility group box 1 complex References: PMID:20826760 Sources: GOC:BHF, GOC:ebc Definition: A protein complex that consists of an alphav-beta3 integrin complex bound to high mobility group box 1 protein.